{
  "term_id": "UNKNOWN:0002",
  "gene": "UniProtKB:Q8N806",
  "gene_name": "Putative E3 ubiquitin-protein ligase UBR7",
  "gene_symbol": "UBR7",
  "term_label": "Unknown biological process"
}